{
  "gene_name": "Megakaryocyte and platelet inhibitory receptor G6b",
  "gene": "UniProtKB:O95866",
  "term_id": "GO:0007596",
  "gene_symbol": "MPIG6B",
  "term_label": "blood coagulation"
}